{
  "gene_name": "Putative methyl-CpG-binding domain protein 3-like 4",
  "term_label": "methyl-CpG binding",
  "gene": "UniProtKB:A6NDZ8",
  "term_id": "GO:0008327",
  "gene_symbol": "MBD3L4"
}